compound eye pigmentation [GO:0048072] (biological process) Sources: GOC:jid Regulation: regulated by regulation of compound eye pigmentation [GO:0048076]; negatively regulated by negative regulation of compound eye pigmentation [GO:0048077]; positively regulated by GO:0048078 Relationships: is a type of eye pigmentation [GO:0048069] Definition: Establishment of a pattern of pigment in the compound eye.